{
  "term_label": "cellular response to glucose starvation",
  "gene_symbol": "PRKAG3",
  "gene_name": "5'-AMP-activated protein kinase subunit gamma-3",
  "gene": "UniProtKB:Q9UGI9",
  "term_id": "GO:0042149"
}